{
  "gene_name": "Secretogranin-1",
  "term_id": "GO:0005615",
  "gene": "UniProtKB:P05060",
  "term_label": "extracellular space",
  "gene_symbol": "CHGB"
}